{
  "gene_symbol": "ATP6V0A1",
  "gene_name": "V-type proton ATPase 116 kDa subunit a 1",
  "gene": "UniProtKB:Q93050",
  "term_label": "vacuolar proton-transporting V-type ATPase complex",
  "term_id": "GO:0016471"
}